{
  "term_label": "regulation of transcription by RNA polymerase II",
  "gene_symbol": "ZNF23",
  "term_id": "GO:0006357",
  "gene": "UniProtKB:P17027",
  "gene_name": "Zinc finger protein 23"
}